histone H3K4me3 reader activity [GO:0140002] (molecular function) Relationships: is a type of histone H3 reader activity [GO:0140006] Definition: A histone reader that recognizes a histone H3 trimethylated at lysine 4. References: PMID:15647753, PMID:23318260 Also known as: H3-K4me3 modified histone binding, H3K4me3 modified histone binding Note: Comment: Note that the residue position corresponds to the canonical human H3 histone (UniProtKB:P84243); this residue is conserved across all eukaryotes. Residue 1 is the first residue following removal of the initiating Methionine (Met). Note that each histone is encoded by multiple genes, and sequences may vary across different genes within an organism.